{
  "term_id": "UNKNOWN:0002",
  "gene_name": "Surfactant-associated protein 2",
  "gene_symbol": "SFTA2",
  "gene": "UniProtKB:Q6UW10",
  "term_label": "Unknown biological process"
}